regulation of sorocarp stalk cell differentiation [GO:0031285] (biological process) References: PMID:4338436 Sources: GOC:kp, GOC:mtg_sensu Subtypes: negative regulation of sorocarp stalk cell differentiation [GO:0031286], positive regulation of sorocarp stalk cell differentiation [GO:0031287] Also known as: regulation of stalk cell differentiation Definition: Any process that modulates the frequency, rate or extent of sorocarp stalk cell differentiation. An example of this process is found in Dictyostelium discoideum. Relationships: is a type of regulation of cell differentiation [GO:0045595]; regulates GO:0031149